response to intra-S DNA damage checkpoint signaling [GO:0072429] (biological process) Relationships: is a type of response to DNA damage checkpoint signaling [GO:0072423] Also known as: intra-S DNA damage checkpoint effector process, response to signal involved in intra-S DNA damage checkpoint Sources: GOC:mtg_cell_cycle Definition: A process that occurs in response to signals generated as a result of intra-S DNA damage checkpoint signaling.